{
  "term_id": "GO:0008465",
  "gene_name": "Glyoxylate reductase_hydroxypyruvate reductase",
  "gene_symbol": "GRHPR",
  "gene": "UniProtKB:Q9UBQ7",
  "term_label": "hydroxypyruvate reductase (NADH) activity"
}